N-formylglutamate deformylase activity [GO:0050129] (molecular function) Definition: Catalysis of the reaction: N-formyl-L-glutamate + H2O = L-glutamate + formate. Also known as: N-formyl-L-glutamate amidohydrolase activity, N-formylglutamate hydrolase activity, beta-citryl-L-glutamate amidase activity, beta-citryl-L-glutamate amidohydrolase activity, beta-citryl-L-glutamate hydrolase activity, beta-citryl-L-glutamate-hydrolyzing enzyme, beta-citrylglutamate amidase activity, formylglutamate deformylase activity Sources: EC:3.5.1.68, RHEA:12476 Relationships: is a type of hydrolase activity, acting on carbon-nitrogen (but not peptide) bonds, in linear amides [GO:0016811]